{
  "term_label": "GTP binding",
  "gene": "UniProtKB:P30793",
  "gene_name": "GTP cyclohydrolase 1",
  "term_id": "GO:0005525",
  "gene_symbol": "GCH1"
}